sphingolipid alpha-glucuronosyltransferase activity [GO:1990482] (molecular function) Also known as: inositol phosphorylceramide glucuronosyltransferase activity Relationships: is a type of UDP-glycosyltransferase activity [GO:0008194] References: PMID:25122154 Sources: GOC:tb Definition: Catalysis of the reaction: UDP-glucuronate + inositol phosphorylceramide (IPC) = UDP + GlcA-IPC.